{
  "gene": "UniProtKB:O15068",
  "term_id": "GO:0005737",
  "term_label": "cytoplasm",
  "gene_symbol": "MCF2L",
  "gene_name": "Guanine nucleotide exchange factor DBS"
}